{
  "term_id": "GO:0006703",
  "term_label": "estrogen biosynthetic process",
  "gene_name": "(3R)-3-hydroxyacyl-CoA dehydrogenase",
  "gene": "UniProtKB:Q92506",
  "gene_symbol": "HSD17B8"
}